negative regulation of Frizzled Nuclear Import pathway [GO:0140712] (biological process) Relationships: is a type of regulation of Frizzled Nuclear Import pathway [GO:0140710]; is a type of negative regulation of non-canonical Wnt signaling pathway [GO:2000051]; negatively regulates GO:0140709 Definition: Any process that stops, prevents, or reduces the frequency, rate or extent of a Frizzled Nuclear Import pathway. Also known as: negative regulation of FNI, negative regulation of Frizzled Nuclear Import Wnt Pathway References: PMID:22510459, PMID:22579286